vitellogenesis [GO:0007296] (biological process) Regulation: regulated by GO:1903186; negatively regulated by GO:1903187; positively regulated by positive regulation of vitellogenesis [GO:1903188] Sources: GOC:dph, ISBN:0879694238 Definition: The production of yolk. Yolk is a mixture of materials used for embryonic nutrition. Relationships: is a type of cytoplasm organization [GO:0007028]; is part of female gamete generation [GO:0007292] Also known as: yolk formation, yolk production